{
  "term_label": "immune response",
  "term_id": "GO:0006955",
  "gene_symbol": "CD209",
  "gene_name": "CD209 antigen",
  "gene": "UniProtKB:Q9NNX6"
}